{
  "gene": "UniProtKB:Q0ZLH3",
  "term_label": "cytoplasm",
  "gene_symbol": "PJVK",
  "term_id": "GO:0005737",
  "gene_name": "Pejvakin"
}